{
  "term_label": "ossification",
  "term_id": "GO:0001503",
  "gene_name": "V-type proton ATPase 116 kDa subunit a 3",
  "gene": "UniProtKB:Q13488",
  "gene_symbol": "TCIRG1"
}